{
  "gene": "UniProtKB:Q9C086",
  "term_id": "GO:0031011",
  "term_label": "Ino80 complex",
  "gene_name": "INO80 complex subunit B",
  "gene_symbol": "INO80B"
}